response to mitotic spindle checkpoint signaling [GO:0072476] (biological process) Sources: GOC:mtg_cell_cycle Also known as: mitotic cell cycle spindle checkpoint effector process, response to mitotic cell cycle spindle checkpoint signaling, response to signal involved in mitotic cell cycle spindle checkpoint Subtypes: response to mitotic cell cycle spindle assembly checkpoint signaling [GO:0072479], response to mitotic cell cycle spindle orientation checkpoint signaling [GO:0072482] Definition: A process that occurs in response to signals generated as a result of mitotic cell cycle spindle checkpoint signaling. Relationships: is a type of response to mitotic cell cycle checkpoint signaling [GO:0072414]; is_a response to spindle checkpoint signaling [GO:0072417]